ventral disc overlap zone [GO:0097592] (CC) Also known as: overlap zone, ventral disk overlap zone Note: Due to the asymmetric nature of the Giardia trophozoite, this term is defined spatially as the trophozoite is viewed from the dorsal side, with the two nuclei dorsal to the ventral disc, and the ventral disc toward the anterior. Relationships: is a type of GO:0110165; is part of GO:0097597; has part ventral disc microtubule array [GO:0097593] Definition: A region of the ventral disc of Giardia species (trophozoite stage) where two portions of the same array of microtubules overlap (the microtubule array makes a complete circle and overlaps on itself). Sources: GOC:giardia